glial cell proliferation [GO:0014009] (biological process) Sources: GOC:ef, ISBN:0878932585 Relationships: is a type of cell population proliferation [GO:0008283]; is part of gliogenesis [GO:0042063] Definition: The multiplication or reproduction of glial cells by cell division, resulting in the expansion of their population. Glial cells exist throughout the nervous system, and include Schwann cells, astrocytes, and oligodendrocytes among others. Regulation: regulated by regulation of glial cell proliferation [GO:0060251]; positively regulated by positive regulation of glial cell proliferation [GO:0060252]; negatively regulated by negative regulation of glial cell proliferation [GO:0060253] Subtypes: Schwann cell proliferation [GO:0014010], microglial cell proliferation [GO:0061518] Also known as: glia proliferation